{
  "gene": "UniProtKB:O15519",
  "term_label": "positive regulation of neuron apoptotic process",
  "term_id": "GO:0043525",
  "gene_name": "CASP8 and FADD-like apoptosis regulator",
  "gene_symbol": "CFLAR"
}